{
  "gene_symbol": "HRH2",
  "term_id": "GO:0005886",
  "gene_name": "Histamine H2 receptor",
  "term_label": "plasma membrane",
  "gene": "UniProtKB:P25021"
}